{
  "gene_name": "Tubulin beta-6 chain",
  "gene": "UniProtKB:Q9BUF5",
  "term_id": "GO:0005874",
  "term_label": "microtubule",
  "gene_symbol": "TUBB6"
}